{
  "gene_name": "Neurotrypsin",
  "term_id": "GO:0004252",
  "gene_symbol": "PRSS12",
  "gene": "UniProtKB:P56730",
  "term_label": "serine-type endopeptidase activity"
}